{
  "gene_name": "Dipeptidase 2",
  "gene": "UniProtKB:Q9H4A9",
  "term_label": "Unknown biological process",
  "term_id": "UNKNOWN:0002",
  "gene_symbol": "DPEP2"
}